{
  "gene_symbol": "HTR3C",
  "term_id": "GO:1902495",
  "gene": "UniProtKB:Q8WXA8",
  "term_label": "transmembrane transporter complex",
  "gene_name": "5-hydroxytryptamine receptor 3C"
}